{
  "gene_name": "CST complex subunit STN1",
  "gene_symbol": "STN1",
  "term_label": "telomeric DNA binding",
  "gene": "UniProtKB:Q9H668",
  "term_id": "GO:0042162"
}